{
  "term_label": "protein localization to plasma membrane",
  "gene_name": "Ankyrin-2",
  "gene": "UniProtKB:Q01484",
  "term_id": "GO:0072659",
  "gene_symbol": "ANK2"
}